{
  "gene_symbol": "PLPBP",
  "gene": "UniProtKB:O94903",
  "term_id": "GO:0005737",
  "term_label": "cytoplasm",
  "gene_name": "Pyridoxal phosphate homeostasis protein"
}